histone H2AX kinase activity [GO:0141003] (molecular function) Subtypes: GO:0035979, histone H2AXY142 kinase activity [GO:0140801] Relationships: is a type of histone kinase activity [GO:0035173] Sources: GOC:bf Definition: Catalysis of the transfer of a phosphate group to a histone variant H2AX.